{
  "gene_name": "Beta-1,4-galactosyltransferase 1",
  "gene_symbol": "B4GALT1",
  "term_label": "beta-N-acetylglucosaminylglycopeptide beta-1,4-galactosyltransferase activity",
  "gene": "UniProtKB:P15291",
  "term_id": "GO:0003831"
}